{
  "gene_name": "Mu-type opioid receptor",
  "term_label": "sensory perception of pain",
  "gene_symbol": "OPRM1",
  "term_id": "GO:0019233",
  "gene": "UniProtKB:P35372"
}